{
  "term_label": "G protein-coupled receptor activity",
  "gene_symbol": "GPR183",
  "term_id": "GO:0004930",
  "gene": "UniProtKB:P32249",
  "gene_name": "G-protein coupled receptor 183"
}